negative regulation of JNK cascade [GO:0046329] (biological process) Definition: Any process that stops, prevents, or reduces the frequency, rate or extent of signal transduction mediated by the JNK cascade. Sources: GOC:bf Also known as: down regulation of JNK cascade, down-regulation of JNK cascade, downregulation of JNK cascade, inhibition of JNK cascade Relationships: is a type of negative regulation of MAPK cascade [GO:0043409]; is a type of regulation of JNK cascade [GO:0046328]; negatively regulates JNK cascade [GO:0007254] Subtypes: negative regulation of JUN kinase activity [GO:0043508]